{
  "term_id": "GO:0005813",
  "gene_name": "Nuclear distribution protein nudE homolog 1",
  "term_label": "centrosome",
  "gene_symbol": "NDE1",
  "gene": "UniProtKB:Q9NXR1"
}